diadenosine pentaphosphate catabolic process [GO:1901907] (biological process) Definition: The chemical reactions and pathways resulting in the breakdown of diadenosine pentaphosphate. Also known as: diadenosine pentaphosphate catabolism, diadenosyl pentaphosphate breakdown, diadenosyl pentaphosphate catabolic process, diadenosyl pentaphosphate catabolism, diadenosyl pentaphosphate degradation References: PMID:10090752 Sources: GOC:TermGenie Relationships: is a type of diadenosine polyphosphate catabolic process [GO:0015961]